{
  "gene_name": "Protein kish-B",
  "term_id": "UNKNOWN:0001",
  "gene_symbol": "TMEM167B",
  "gene": "UniProtKB:Q9NRX6",
  "term_label": "Unknown molecular function"
}